cytoplasmic translational elongation through polyproline stretches [GO:0097622] (biological process) Relationships: is a type of cytoplasmic translational elongation [GO:0002182] References: PMID:24923804 Sources: GOC:mcc Regulation: regulated by regulation of cytoplasmic translational elongation through polyproline stretches [GO:1903270]; negatively regulated by negative regulation of cytoplasmic translational elongation through polyproline stretches [GO:1903271]; positively regulated by positive regulation of cytoplasmic translational elongation through polyproline stretches [GO:1903272] Definition: The successive addition of amino acid residues to a nascent polypeptide chain, proceeding through regions of multiple repeated proline codons, during protein biosynthesis in the cytoplasm.